{
  "term_label": "plasma membrane",
  "gene_name": "Olfactory receptor 6A2",
  "term_id": "GO:0005886",
  "gene": "UniProtKB:O95222",
  "gene_symbol": "OR6A2"
}